{
  "gene_symbol": "ZFHX3",
  "term_label": "nucleus",
  "gene": "UniProtKB:Q15911",
  "term_id": "GO:0005634",
  "gene_name": "Zinc finger homeobox protein 3"
}